{
  "term_label": "positive regulation of canonical Wnt signaling pathway",
  "term_id": "GO:0090263",
  "gene": "UniProtKB:O95271",
  "gene_name": "Poly [ADP-ribose] polymerase tankyrase-1",
  "gene_symbol": "TNKS"
}